regulation of actin filament organization [GO:0110053] (BP) Subtypes: GO:0008064, regulation of actin filament bundle assembly [GO:0032231], regulation of actin nucleation [GO:0051125], regulation of actin filament annealing [GO:0110054] Definition: Any process that modulates the frequency, rate or extent of actin filament organization. Sources: GOC:kmv Relationships: is a type of regulation of actin cytoskeleton organization [GO:0032956]; is a type of regulation of supramolecular fiber organization [GO:1902903]; regulates actin filament organization [GO:0007015]